filamentous growth of a population of unicellular organisms [GO:0044182] (biological process) Sources: GOC:mtg_cambridge_2009 Subtypes: filamentous growth of a population of unicellular organisms in response to heat [GO:0036168], filamentous growth of a population of unicellular organisms in response to starvation [GO:0036170], filamentous growth of a population of unicellular organisms in response to chemical stimulus [GO:0036171], GO:0036177, filamentous growth of a population of unicellular organisms in response to biotic stimulus [GO:0036180], growth of unicellular organism as a thread of attached cells [GO:0070783] Relationships: is a type of filamentous growth [GO:0030447] Regulation: RO_0002211 by regulation of filamentous growth of a population of unicellular organisms [GO:1900428]; negatively regulated by negative regulation of filamentous growth of a population of unicellular organisms [GO:1900429]; positively regulated by positive regulation of filamentous growth of a population of unicellular organisms [GO:1900430] Definition: The process in which a group of unicellular organisms grow in a threadlike, filamentous shape.